{
  "term_id": "UNKNOWN:0001",
  "gene_symbol": "KRTAP21-3",
  "gene": "UniProtKB:Q3LHN1",
  "term_label": "Unknown molecular function",
  "gene_name": "Keratin-associated protein 21-3"
}